butyrate kinase activity [GO:0047761] (MF) Also known as: ATP:butanoate 1-phosphotransferase activity Relationships: is a type of GO:0016301; is a type of phosphotransferase activity, carboxyl group as acceptor [GO:0016774] Definition: Catalysis of the reaction: ATP + butanoate = ADP + butanoyl phosphate + H+. Sources: EC:2.7.2.7, RHEA:13585